Sec61 translocon complex [GO:0005784] (cellular component) Definition: A translocon complex that contains a core heterotrimer of conserved alpha, beta and gamma subunits, and may contain additional proteins (translocon-associated proteins or TRAPs); in budding yeast the core proteins are Sec61p, Sbh1p, and Sss1p. The Sec61 translocon complex functions in cotranslational and posttranslational translocation events. Also known as: Sec61p-Sbh1p-Sss1p complex References: PMID:18166647, PMID:32820719, PMID:33960686 Sources: GOC:mah Relationships: is a type of translocon complex [GO:0071256]